{
  "term_label": "microtubule binding",
  "gene": "UniProtKB:Q9P2P6",
  "gene_name": "StAR-related lipid transfer protein 9",
  "gene_symbol": "STARD9",
  "term_id": "GO:0008017"
}